viral terminase complex [GO:0043493] (cellular component) Also known as: virus terminase complex, phage terminase complex Definition: A complex of a large and small subunit which catalyze the packaging of DNA into viral heads. Note that not all viral terminases have this structure, some exist as single polypeptides. References: PMID:18687036 Sources: GOC:bf, GOC:bm, GOC:jl, GOC:mlg Relationships: is a type of protein-containing complex [GO:0032991]